{
  "gene_name": "Fumarate hydratase, mitochondrial",
  "gene_symbol": "FH",
  "term_label": "fumarate hydratase activity",
  "term_id": "GO:0004333",
  "gene": "UniProtKB:P07954"
}